{
  "gene_symbol": "SLC12A2",
  "gene_name": "Solute carrier family 12 member 2",
  "term_label": "sodium:potassium:chloride symporter activity",
  "term_id": "GO:0008511",
  "gene": "UniProtKB:P55011"
}